{
  "gene_name": "Microtubule-associated protein 9",
  "gene_symbol": "MAP9",
  "term_id": "GO:0000235",
  "term_label": "astral microtubule",
  "gene": "UniProtKB:Q49MG5"
}